{
  "gene": "UniProtKB:Q9Y5E4",
  "gene_symbol": "PCDHB5",
  "term_label": "plasma membrane",
  "term_id": "GO:0005886",
  "gene_name": "Protocadherin beta-5"
}